{
  "gene_symbol": "OR5D14",
  "term_label": "Unknown cellular component",
  "gene_name": "Olfactory receptor 5D14",
  "gene": "UniProtKB:Q8NGL3",
  "term_id": "UNKNOWN:0003"
}